{
  "gene_symbol": "GADD45GIP1",
  "gene_name": "Large ribosomal subunit protein mL64",
  "gene": "UniProtKB:Q8TAE8",
  "term_label": "Unknown biological process",
  "term_id": "UNKNOWN:0002"
}